{
  "gene_name": "Keratin-associated protein 9-6",
  "gene_symbol": "KRTAP9-6",
  "term_label": "Unknown molecular function",
  "term_id": "UNKNOWN:0001",
  "gene": "UniProtKB:A8MVA2"
}